{
  "term_id": "GO:0005886",
  "gene_symbol": "KLRC2",
  "gene_name": "NKG2-C type II integral membrane protein",
  "term_label": "plasma membrane",
  "gene": "UniProtKB:P26717"
}